glutamine metabolic process [GO:0006541] (BP) Relationships: is a type of glutamine family amino acid metabolic process [GO:0009064] Subtypes: glutamine biosynthetic process [GO:0006542], L-glutamine catabolic process [GO:0006543], ammonia assimilation cycle [GO:0019676], cyclization of glutamine involved in intein-mediated protein splicing [GO:0019802] Also known as: glutamine metabolism Definition: The chemical reactions and pathways involving glutamine, 2-amino-4-carbamoylbutanoic acid. Sources: GOC:ai